negative regulation of free ubiquitin chain polymerization [GO:1904543] (biological process) Relationships: is a type of negative regulation of protein polymerization [GO:0032272]; is a type of regulation of free ubiquitin chain polymerization [GO:1904542]; negatively regulates free ubiquitin chain polymerization [GO:0010994] References: PMID:24660806 Sources: GOC:PARL, GOC:TermGenie, GOC:pad, GO_REF:0000058 Note: An example of this is PARK2 in human (UniProt symbol O60260) in PMID:24660806 (inferred from mutant phenotype). Definition: Any process that stops, prevents or reduces the frequency, rate or extent of free ubiquitin chain polymerization. Also known as: down regulation of free ubiquitin chain polymerization, down-regulation of free ubiquitin chain polymerization, downregulation of free ubiquitin chain polymerization, inhibition of free ubiquitin chain polymerization